{
  "gene": "UniProtKB:Q96RA2",
  "term_id": "GO:0005886",
  "gene_symbol": "OR7D2",
  "term_label": "plasma membrane",
  "gene_name": "Olfactory receptor 7D2"
}